{
  "term_label": "extracellular space",
  "gene": "UniProtKB:P20742",
  "term_id": "GO:0005615",
  "gene_symbol": "PZP",
  "gene_name": "Pregnancy zone protein"
}